{
  "term_label": "plasma membrane",
  "term_id": "GO:0005886",
  "gene_symbol": "CDC42EP1",
  "gene": "UniProtKB:Q00587",
  "gene_name": "Cdc42 effector protein 1"
}